{
  "gene_symbol": "LRRFIP2",
  "term_label": "Unknown biological process",
  "gene": "UniProtKB:Q9Y608",
  "gene_name": "Leucine-rich repeat flightless-interacting protein 2",
  "term_id": "UNKNOWN:0002"
}